{
  "gene_name": "Sterol 26-hydroxylase, mitochondrial",
  "gene_symbol": "CYP27A1",
  "term_label": "cholesterol 26-hydroxylase activity",
  "term_id": "GO:0031073",
  "gene": "UniProtKB:Q02318"
}